protein localization to tricellular tight junction [GO:0061833] (biological process) Definition: A process in which a protein is transported to, or maintained in, a location within a tricellular tight junction. Relationships: is a type of protein localization to cell-cell junction [GO:0150105] References: PMID:24889144